{
  "gene_symbol": "TUBB8",
  "term_id": "GO:0005737",
  "term_label": "cytoplasm",
  "gene": "UniProtKB:Q3ZCM7",
  "gene_name": "Tubulin beta-8 chain"
}